negative regulation of sodium ion import across plasma membrane [GO:1903783] (biological process) Also known as: down regulation of sodium ion import across plasma membrane, down-regulation of sodium ion import across plasma membrane, downregulation of sodium ion import across plasma membrane, inhibition of sodium ion import across plasma membrane Definition: Any process that stops, prevents or reduces the frequency, rate or extent of sodium ion import across the plasma membrane. Relationships: is a type of negative regulation of sodium ion transmembrane transport [GO:1902306]; is a type of regulation of sodium ion import across plasma membrane [GO:1903782]; negatively regulates GO:0098719 References: PMID:19376779 Sources: GOC:BHF, GOC:TermGenie, GOC:mtg_cardiac_conduct_nov11, GOC:nc, GO_REF:0000058